{
  "gene_symbol": "NXPE3",
  "term_id": "UNKNOWN:0001",
  "gene_name": "NXPE family member 3",
  "gene": "UniProtKB:Q969Y0",
  "term_label": "Unknown molecular function"
}